orotate:monoatomic anion antiporter activity [GO:0140812] (molecular function) Definition: Enables the transfer of a solute or solutes from one side of a membrane to the other according to the reaction: orotate(out) + anion (in) = orotate (in) + anion (out). References: PMID:21350910, PMID:35144162 Also known as: orotate:anion antiporter activity, orotate:organic anion antiporter activity Relationships: is a type of monoatomic anion transmembrane transporter activity [GO:0008509]; is a type of antiporter activity [GO:0015297]; is a type of GO:0015355